{
  "term_label": "plasma membrane",
  "gene": "UniProtKB:P0DN77",
  "gene_symbol": "OPN1MW2",
  "gene_name": "Medium-wave-sensitive opsin 2",
  "term_id": "GO:0005886"
}